{
  "gene_symbol": "EDA",
  "term_id": "GO:0042476",
  "gene_name": "Ectodysplasin-A",
  "term_label": "odontogenesis",
  "gene": "UniProtKB:Q92838"
}